{
  "term_id": "GO:1902476",
  "gene": "UniProtKB:A0AV02",
  "term_label": "chloride transmembrane transport",
  "gene_symbol": "SLC12A8",
  "gene_name": "Solute carrier family 12 member 8"
}